{
  "term_label": "Unknown molecular function",
  "gene": "UniProtKB:Q96T51",
  "gene_symbol": "RUFY1",
  "term_id": "UNKNOWN:0001",
  "gene_name": "RUN and FYVE domain-containing protein 1"
}